{
  "gene": "UniProtKB:Q16666",
  "term_id": "GO:0005730",
  "gene_name": "Gamma-interferon-inducible protein 16",
  "term_label": "nucleolus",
  "gene_symbol": "IFI16"
}